{
  "term_id": "UNKNOWN:0003",
  "gene_symbol": "MGAM2",
  "gene": "UniProtKB:Q2M2H8",
  "gene_name": "Probable maltase-glucoamylase 2",
  "term_label": "Unknown cellular component"
}